{
  "gene": "UniProtKB:P48380",
  "gene_name": "Transcription factor RFX3",
  "term_label": "nucleus",
  "gene_symbol": "RFX3",
  "term_id": "GO:0005634"
}